symbiont-mediated suppression of host NF-kappaB cascade [GO:0085034] (biological process) Also known as: disruption of host I-kappaB kinase/NF-kappaB cascade, negative regulation by symbiont of host I-kappaB kinase/NF-kappaB cascade, suppression by symbiont of host I-kappaB kinase/NF-kappaB cascade, disruption of host canonical NF-kappaB cascade, symbiont-mediated suppression of host canonical NF-kappaB cascade References: PMID:18250452, PMID:22442494, PMID:24648522, PMID:33567255 Definition: A process in which a symbiont interferes with, inhibits or disrupts an NF-kappaB-mediated signaling cascade in its host organism. The host is defined as the larger of the organisms involved in a symbiotic interaction. Relationships: is a type of symbiont-mediated suppression of host signal transduction pathway [GO:0052029]; is a type of symbiont-mediated perturbation of host NF-kappaB cascade [GO:0085032]